regulation of glucose metabolic process [GO:0010906] (biological process) Definition: Any process that modulates the rate, frequency or extent of glucose metabolism. Glucose metabolic processes are the chemical reactions and pathways involving glucose, the aldohexose gluco-hexose. Subtypes: regulation of gluconeogenesis [GO:0006111], positive regulation of glucose metabolic process [GO:0010907], regulation of glucose catabolic process to lactate via pyruvate [GO:1904023] Sources: GOC:BHF, GOC:tb Relationships: is a type of regulation of carbohydrate metabolic process [GO:0006109]; is a type of regulation of small molecule metabolic process [GO:0062012]; regulates glucose metabolic process [GO:0006006] Also known as: regulation of glucose metabolism